phosphatidylglycerol lysyltransferase activity [GO:0050071] (molecular function) Relationships: is a type of aminoacyltransferase activity [GO:0016755] Sources: EC:2.3.2.3 Also known as: lysyltransferase activity, lysylphosphatidylglycerol synthase activity Definition: Catalysis of the reaction: 1,2-diacyl-sn-glycero-3-phospho-(1'-sn-glycerol) + L-lysyl-tRNA(Lys) = 1,2-diacyl-sn-glycero-3-phospho-1'-(3'-O-L-lysyl)-sn-glycerol + tRNA(Lys).